{
  "gene_symbol": "POSTN",
  "gene": "UniProtKB:Q15063",
  "term_id": "GO:0005615",
  "term_label": "extracellular space",
  "gene_name": "Periostin"
}